oxidoreductase activity, acting on CH or CH2 groups, disulfide as acceptor [GO:0016728] (MF) Subtypes: ribonucleoside-triphosphate reductase (thioredoxin) activity [GO:0008998], GO:0047057, vitamin-K-epoxide reductase (warfarin-insensitive) activity [GO:0047058], ribonucleoside-diphosphate reductase activity [GO:0061731] Relationships: is a type of oxidoreductase activity, acting on CH or CH2 groups [GO:0016725] Also known as: oxidoreductase activity, acting on CH or CH2 groups, disulphide as acceptor Definition: Catalysis of an oxidation-reduction (redox) reaction in which a CH2 group acts as a hydrogen or electron donor and reduces a disulfide group. Sources: GOC:ai